host bacteroid-containing symbiosome [GO:0043663] (cellular component) Sources: GOC:cc Definition: A symbiosome containing any of various structurally modified bacteria, such as those occurring on the root nodules of leguminous plants, of a host cell. Relationships: is a type of host symbiosome [GO:0043658]